negative regulation of blood microparticle formation [GO:2000333] (biological process) Definition: Any process that stops, prevents or reduces the frequency, rate or extent of blood microparticle formation. Relationships: is a type of negative regulation of developmental process [GO:0051093]; is a type of negative regulation of cellular component organization [GO:0051129]; is a type of regulation of blood microparticle formation [GO:2000332]; negatively regulates GO:0072564 Sources: GOC:BHF, GOC:mah Also known as: negative regulation of microparticle generation, negative regulation of microparticle release Subtypes: negative regulation of endothelial microparticle formation [GO:2000336]